{
  "term_id": "GO:0005737",
  "gene": "UniProtKB:P38646",
  "term_label": "cytoplasm",
  "gene_name": "Stress-70 protein, mitochondrial",
  "gene_symbol": "HSPA9"
}